{
  "gene_name": "Neurogenic locus notch homolog protein 1",
  "term_id": "GO:0005886",
  "term_label": "plasma membrane",
  "gene_symbol": "NOTCH1",
  "gene": "UniProtKB:P46531"
}